curli secretion complex [GO:0062155] (cellular component) References: PMID:25219853 Definition: A protein-containing complex that serves as a channel for the secretion of curli. Curli are a fibers that serve as a major component of the extracellular matrix of pellicle biofilms. Relationships: is a type of transmembrane transporter complex [GO:1902495]; is part of cell outer membrane [GO:0009279]